{
  "gene_name": "Protein SGT1 homolog",
  "term_id": "UNKNOWN:0003",
  "gene_symbol": "SUGT1",
  "term_label": "Unknown cellular component",
  "gene": "UniProtKB:Q9Y2Z0"
}